{
  "gene": "UniProtKB:Q8NDY6",
  "gene_symbol": "BHLHE23",
  "term_label": "nucleus",
  "gene_name": "Class E basic helix-loop-helix protein 23",
  "term_id": "GO:0005634"
}